regulation of presynapse assembly [GO:1905606] (biological process) Definition: Any process that modulates the frequency, rate or extent of presynapse assembly. References: PMID:25533483 Sources: GOC:PARL, GOC:TermGenie, GOC:bc, GO_REF:0000058 Also known as: regulation of presynapse biogenesis, regulation of presynaptic terminal assembly Relationships: is a type of regulation of synapse assembly [GO:0051963]; is_a regulation of presynapse organization [GO:0099174]; regulates presynapse assembly [GO:0099054] Subtypes: negative regulation of presynapse assembly [GO:1905607], positive regulation of presynapse assembly [GO:1905608]